glycosaminoglycan binding [GO:0005539] (molecular function) Subtypes: hyaluronic acid binding [GO:0005540], GO:0008201, chondroitin sulfate binding [GO:0035374], GO:0042834, GO:1904399 Sources: GOC:jl, ISBN:0198506732 Definition: Binding to a glycan (polysaccharide) containing a substantial proportion of aminomonosaccharide residues. Relationships: is a type of carbohydrate derivative binding [GO:0097367]